{
  "gene_symbol": "INCENP",
  "gene_name": "Inner centromere protein",
  "term_label": "nucleus",
  "gene": "UniProtKB:Q9NQS7",
  "term_id": "GO:0005634"
}